{
  "gene": "UniProtKB:O43143",
  "term_label": "Unknown biological process",
  "gene_symbol": "DHX15",
  "gene_name": "ATP-dependent RNA helicase DHX15",
  "term_id": "UNKNOWN:0002"
}